tight junction disassembly [GO:1905071] (biological process) Definition: The disaggregation of an tight junction into its constituent components. References: PMID:18718461 Sources: GOC:BHF, GOC:TermGenie, GOC:rl, GO_REF:0000079 Also known as: occluding cell junction disassembly, occluding junction disassembly Relationships: is a type of tight junction organization [GO:0120193]; is a type of cell-cell junction disassembly [GO:0150147] Subtypes: tricellular tight junction disassembly [GO:1904275] Regulation: regulated by GO:1905073; negatively regulated by GO:1905074; RO_0002213 by positive regulation of tight junction disassembly [GO:1905075]